{
  "gene_name": "Thrombospondin-type laminin G domain and EAR repeat-containing protein",
  "gene": "UniProtKB:Q8WU66",
  "term_label": "Unknown cellular component",
  "gene_symbol": "TSPEAR",
  "term_id": "UNKNOWN:0003"
}